{
  "gene_symbol": "OR52H1",
  "term_label": "plasma membrane",
  "gene_name": "Olfactory receptor 52H1",
  "term_id": "GO:0005886",
  "gene": "UniProtKB:Q8NGJ2"
}